{
  "term_label": "removal of superoxide radicals",
  "term_id": "GO:0019430",
  "gene_name": "Extracellular superoxide dismutase [Cu-Zn]",
  "gene": "UniProtKB:P08294",
  "gene_symbol": "SOD3"
}